regulation of raffinose metabolic process [GO:0080091] (biological process) Definition: Any process that modulates the frequency, rate or extent of the chemical reactions and pathways involving raffinose. Relationships: is a type of regulation of carbohydrate metabolic process [GO:0006109]; regulates GO:0033530 References: PMID:19211694 Subtypes: regulation of raffinose biosynthetic process [GO:1900091]